{
  "gene_name": "Carboxypeptidase Q",
  "gene": "UniProtKB:Q9Y646",
  "gene_symbol": "CPQ",
  "term_id": "GO:0006590",
  "term_label": "thyroid hormone generation"
}